negative regulation of sequestering of calcium ion [GO:0051283] (biological process) Sources: GOC:ai Also known as: down regulation of sequestering of calcium ion, down-regulation of sequestering of calcium ion, downregulation of sequestering of calcium ion, negative regulation of calcium ion (Ca2+) retention, negative regulation of calcium ion (Ca2+) sequestering, negative regulation of calcium ion (Ca2+) sequestration, negative regulation of calcium ion (Ca2+) storage, negative regulation of retention of calcium ion (Ca2+), negative regulation of sequestering of calcium ion (Ca2+), negative regulation of sequestration of calcium ion (Ca2+), negative regulation of storage of calcium ion (Ca2+), inhibition of sequestering of calcium ion Subtypes: GO:0051209 Definition: Any process that stops, prevents, or reduces the frequency, rate or extent of the binding or confining calcium ions such that they are separated from other components of a biological system. Relationships: is a type of GO:0048523; is a type of regulation of sequestering of calcium ion [GO:0051282]; negatively regulates sequestering of calcium ion [GO:0051208]